{
  "gene_symbol": "SLC32A1",
  "gene_name": "Vesicular inhibitory amino acid transporter",
  "term_label": "glycine transport",
  "gene": "UniProtKB:Q9H598",
  "term_id": "GO:0015816"
}